rhombomere 3 structural organization [GO:0021659] (biological process) Also known as: rhombomere 3 structural organisation Relationships: is a type of GO:0021595; is part of rhombomere 3 morphogenesis [GO:0021658] Definition: The process that contributes to creating the structural organization of rhombomere 3. This process pertains to the physical shaping of a rudimentary structure. Rhombomeres are transverse segments of the developing rhombencephalon. Rhombomeres are lineage restricted, express different genes from one another, and adopt different developmental fates. Rhombomeres are numbered in an anterior to posterior order. Sources: GOC:cls, GOC:dgh, GOC:dph, GOC:jid, GO_REF:0000021